{
  "gene_symbol": "MAD1L1",
  "term_id": "GO:0072686",
  "gene": "UniProtKB:Q9Y6D9",
  "term_label": "mitotic spindle",
  "gene_name": "Mitotic spindle assembly checkpoint protein MAD1"
}